{
  "term_id": "GO:0045659",
  "gene_name": "Phosphatidylinositol 3,4,5-trisphosphate 5-phosphatase 1",
  "term_label": "negative regulation of neutrophil differentiation",
  "gene": "UniProtKB:Q92835",
  "gene_symbol": "INPP5D"
}